{
  "gene": "UniProtKB:Q695T7",
  "gene_symbol": "SLC6A19",
  "term_id": "GO:0015804",
  "gene_name": "Sodium-dependent neutral amino acid transporter B(0)AT1",
  "term_label": "neutral amino acid transport"
}